{
  "term_label": "Unknown molecular function",
  "gene_name": "Putative uncharacterized protein encoded by LINC00588",
  "gene_symbol": "LINC00588",
  "gene": "UniProtKB:Q9Y4M8",
  "term_id": "UNKNOWN:0001"
}